{
  "gene_name": "Uncharacterized protein C12orf40",
  "term_id": "UNKNOWN:0001",
  "gene": "UniProtKB:Q86WS4",
  "gene_symbol": "C12orf40",
  "term_label": "Unknown molecular function"
}